{
  "gene_symbol": "GPR137B",
  "gene": "UniProtKB:O60478",
  "term_label": "negative regulation of bone resorption",
  "term_id": "GO:0045779",
  "gene_name": "Integral membrane protein GPR137B"
}